post-embryonic anterior midgut (ectodermal) morphogenesis [GO:0048616] (biological process) Sources: GOC:jid, GOC:rc Relationships: is a type of post-embryonic animal morphogenesis [GO:0009886]; is part of anterior midgut (ectodermal) morphogenesis [GO:0007441]; is part of post-embryonic ectodermal digestive tract morphogenesis [GO:0048614] Definition: The process in which the anatomical structures of the anterior midgut (ectodermal) are generated and organized, during the post-embryonic phase.